{
  "term_id": "GO:0000981",
  "gene_name": "Ski-like protein",
  "gene": "UniProtKB:P12757",
  "term_label": "DNA-binding transcription factor activity, RNA polymerase II-specific",
  "gene_symbol": "SKIL"
}